{
  "term_label": "exocytic vesicle",
  "gene_name": "Synaptotagmin-15B",
  "term_id": "GO:0070382",
  "gene_symbol": "SYT15B",
  "gene": "UniProtKB:X6R8R1"
}